{
  "term_label": "regulation of actin cytoskeleton organization",
  "gene": "UniProtKB:P52803",
  "term_id": "GO:0032956",
  "gene_name": "Ephrin-A5",
  "gene_symbol": "EFNA5"
}